trimethylamine-N-oxide reductase (cytochrome c) complex [GO:1904852] (cellular component) References: PMID:11056172 Sources: GOC:TermGenie, GOC:bhm, GO_REF:0000088 Relationships: is a type of oxidoreductase complex [GO:1990204] Definition: A protein complex which is capable of trimethylamine-N-oxide reductase (cytochrome c) activity. Note: An example of this is TorA in E. coli (UniProt ID P33225) in PMID:11056172 (inferred from direct assay).